{
  "gene": "UniProtKB:P55285",
  "gene_symbol": "CDH6",
  "term_id": "GO:0016477",
  "term_label": "cell migration",
  "gene_name": "Cadherin-6"
}